{
  "gene_name": "Nischarin",
  "gene": "UniProtKB:Q9Y2I1",
  "term_id": "UNKNOWN:0001",
  "term_label": "Unknown molecular function",
  "gene_symbol": "NISCH"
}